{
  "gene_name": "GRB2-associated-binding protein 4",
  "term_label": "transmembrane receptor protein tyrosine kinase adaptor activity",
  "term_id": "GO:0005068",
  "gene_symbol": "GAB4",
  "gene": "UniProtKB:Q2WGN9"
}